{
  "term_id": "GO:0006357",
  "gene_symbol": "SOX13",
  "term_label": "regulation of transcription by RNA polymerase II",
  "gene_name": "Transcription factor SOX-13",
  "gene": "UniProtKB:Q9UN79"
}